regulation of Ral protein signal transduction [GO:0032485] (biological process) Definition: Any process that modulates the frequency, rate or extent of Ral protein signal transduction. Relationships: is a type of regulation of small GTPase mediated signal transduction [GO:0051056]; regulates Ral protein signal transduction [GO:0032484] Sources: GOC:mah